{
  "term_id": "GO:0001947",
  "gene": "UniProtKB:Q9UMR3",
  "term_label": "heart looping",
  "gene_symbol": "TBX20",
  "gene_name": "T-box transcription factor TBX20"
}